{
  "term_id": "GO:0005654",
  "term_label": "nucleoplasm",
  "gene_symbol": "SUGP2",
  "gene": "UniProtKB:Q8IX01",
  "gene_name": "SURP and G-patch domain-containing protein 2"
}